{
  "term_id": "UNKNOWN:0003",
  "gene_name": "Molybdenum cofactor sulfurase",
  "gene_symbol": "MOCOS",
  "term_label": "Unknown cellular component",
  "gene": "UniProtKB:Q96EN8"
}